positive regulation of hematopoietic stem cell differentiation [GO:1902038] (biological process) References: PMID:23403623 Sources: GOC:TermGenie Definition: Any process that activates or increases the frequency, rate or extent of hematopoietic stem cell differentiation. Relationships: is_a positive regulation of hematopoietic progenitor cell differentiation [GO:1901534]; is a type of regulation of hematopoietic stem cell differentiation [GO:1902036]; is a type of GO:2000738; RO_0002213 hematopoietic stem cell differentiation [GO:0060218] Also known as: positive regulation of haematopoietic stem cell differentiation, positive regulation of haemopoietic stem cell differentiation, positive regulation of hemopoietic stem cell differentiation, up regulation of haematopoietic stem cell differentiation, up regulation of haemopoietic stem cell differentiation, up regulation of hematopoietic stem cell differentiation, up regulation of hemopoietic stem cell differentiation, up-regulation of haematopoietic stem cell differentiation, up-regulation of haemopoietic stem cell differentiation, up-regulation of hematopoietic stem cell differentiation, up-regulation of hemopoietic stem cell differentiation, upregulation of haematopoietic stem cell differentiation, upregulation of haemopoietic stem cell differentiation, upregulation of hematopoietic stem cell differentiation, upregulation of hemopoietic stem cell differentiation, activation of haematopoietic stem cell differentiation, activation of haemopoietic stem cell differentiation, activation of hematopoietic stem cell differentiation, activation of hemopoietic stem cell differentiation